cytoplasmic pattern recognition receptor signaling pathway [GO:0002753] (BP) Also known as: cytoplasmic PRR signaling pathway, cytoplasmic pathogen receptor signaling pathway, cytoplasmic pattern recognition receptor signalling pathway, cytosolic PAMP receptor signaling pathway, cytosolic pattern recognition receptor signaling pathway, cytoplasmic caspase-recruiting domain (CARD) helicase signaling pathway Subtypes: endosomal pattern recognition receptor signaling pathway [GO:0002754], nucleotide-binding domain, leucine rich repeat containing receptor signaling pathway [GO:0035872], GO:0039529, MDA-5 signaling pathway [GO:0039530], endolysosomal toll-like receptor signaling pathway [GO:0140894], GO:0140896, inflammasome-mediated signaling pathway [GO:0141084] Relationships: is a type of pattern recognition receptor signaling pathway [GO:0002221]; is a type of intracellular receptor signaling pathway [GO:0030522]; has part positive regulation of cytokine production [GO:0001819] Note: This term should be used for annotation when it is not known which cytoplasmic pattern recognition receptor (PRR) has been activated. If the PRR is known, consider instead the child terms. The RIG-like family is composed of at least RIG-I (retinoic acid inducible gene I; also known as DDX58), melanoma differentiation-associated gene 5 (MDA5; also known as helicard or IFIH1) and LGP2. Regulation: RO_0002211 by regulation of cytoplasmic pattern recognition receptor signaling pathway [GO:0039531]; RO_0002212 by negative regulation of cytoplasmic pattern recognition receptor signaling pathway [GO:0039532] References: PMID:15199967, PMID:17328678, PMID:18272355, PMID:19531363, PMID:21187438 Sources: GOC:add, GOC:ar, ISBN:0781735149 Definition: The series of molecular signals initiated by the binding of a ligand from another organism to a cytoplasmic pattern recognition receptor (PRR). PRRs bind pathogen-associated molecular pattern (PAMPs), structures conserved among microbial species.